{
  "gene_symbol": "ITGAL",
  "term_id": "GO:0009986",
  "gene_name": "Integrin alpha-L",
  "gene": "UniProtKB:P20701",
  "term_label": "cell surface"
}